{
  "term_id": "UNKNOWN:0002",
  "gene_symbol": "BPNT1",
  "term_label": "Unknown biological process",
  "gene_name": "3'(2'),5'-bisphosphate nucleotidase 1",
  "gene": "UniProtKB:O95861"
}